{
  "gene_name": "2-5A-dependent ribonuclease",
  "term_id": "GO:0004540",
  "term_label": "RNA nuclease activity",
  "gene": "UniProtKB:Q05823",
  "gene_symbol": "RNASEL"
}